{
  "term_label": "Unknown cellular component",
  "gene": "UniProtKB:Q9NZJ4",
  "gene_name": "Sacsin",
  "gene_symbol": "SACS",
  "term_id": "UNKNOWN:0003"
}